negative regulation of Fas signaling pathway [GO:1902045] (biological process) Also known as: down regulation of Apo-1 signaling pathway, down regulation of CD95 signaling pathway, down regulation of Fas receptor signaling pathway, down regulation of Fas signaling pathway, down regulation of FasR signaling pathway, down-regulation of Apo-1 signaling pathway, down-regulation of CD95 signaling pathway, down-regulation of Fas receptor signaling pathway, down-regulation of Fas signaling pathway, down-regulation of FasR signaling pathway, downregulation of Apo-1 signaling pathway, downregulation of CD95 signaling pathway, downregulation of Fas receptor signaling pathway, downregulation of Fas signaling pathway, downregulation of FasR signaling pathway, negative regulation of Apo-1 signaling pathway, negative regulation of CD95 signaling pathway, negative regulation of Fas receptor signaling pathway, negative regulation of FasR signaling pathway, down regulation of FAS ligand-Fas signaling pathway, down regulation of Fas-FasL signaling pathway, down-regulation of FAS ligand-Fas signaling pathway, down-regulation of Fas-FasL signaling pathway, downregulation of FAS ligand-Fas signaling pathway, downregulation of Fas-FasL signaling pathway, inhibition of Apo-1 signaling pathway, inhibition of CD95 signaling pathway, inhibition of FAS ligand-Fas signaling pathway, inhibition of Fas receptor signaling pathway, inhibition of Fas signaling pathway, inhibition of Fas-FasL signaling pathway, inhibition of FasR signaling pathway, negative regulation of FAS ligand-Fas signaling pathway, negative regulation of Fas-FasL signaling pathway, down regulation of FasL signaling pathway, down-regulation of FasL signaling pathway, downregulation of FasL signaling pathway, inhibition of FasL signaling pathway, negative regulation of FasL signaling pathway Definition: Any process that stops, prevents or reduces the frequency, rate or extent of Fas signaling pathway. Relationships: is_a GO:0009968; is a type of GO:1902044; RO_0002212 Fas signaling pathway [GO:0036337] References: PMID:17245429 Sources: GOC:TermGenie